{
  "term_id": "UNKNOWN:0002",
  "term_label": "Unknown biological process",
  "gene_symbol": "COL5A1-AS1",
  "gene_name": "Putative uncharacterized protein encoded by COL5A1-AS1",
  "gene": "UniProtKB:Q5SY13"
}